{
  "gene_name": "Proline-rich protein 3",
  "term_label": "PTW/PP1 phosphatase complex",
  "gene_symbol": "PRR3",
  "gene": "UniProtKB:P79522",
  "term_id": "GO:0072357"
}